{
  "term_label": "meiotic sister chromatid cohesion",
  "gene": "UniProtKB:Q13362",
  "term_id": "GO:0051177",
  "gene_name": "Serine_threonine-protein phosphatase 2A 56 kDa regulatory subunit gamma isoform",
  "gene_symbol": "PPP2R5C"
}